{
  "term_label": "mitochondrial matrix",
  "gene_name": "Acyl-coenzyme A synthetase ACSM6, mitochondrial",
  "term_id": "GO:0005759",
  "gene_symbol": "ACSM6",
  "gene": "UniProtKB:Q6P461"
}